central plaque of spindle pole body [GO:0005823] (cellular component) Subtypes: central plaque of mitotic spindle pole body [GO:0061493] Relationships: is a type of cellular anatomical structure [GO:0110165]; is part of spindle pole body [GO:0005816] Sources: ISBN:0879693568 Definition: One of three laminate structures that form the spindle pole body; the central plaque is embedded in the nuclear envelope.